{
  "term_id": "GO:0005829",
  "term_label": "cytosol",
  "gene_symbol": "RNF10",
  "gene": "UniProtKB:Q8N5U6",
  "gene_name": "E3 ubiquitin-protein ligase RNF10"
}